{
  "term_id": "GO:0043266",
  "gene_symbol": "DRD2",
  "term_label": "regulation of potassium ion transport",
  "gene_name": "D(2) dopamine receptor",
  "gene": "UniProtKB:P14416"
}